{
  "term_label": "Unknown biological process",
  "term_id": "UNKNOWN:0002",
  "gene_symbol": "A0A8V8TPP0",
  "gene_name": "Uncharacterized protein",
  "gene": "UniProtKB:A0A8V8TPP0"
}